{
  "gene": "UniProtKB:Q13131",
  "gene_name": "5'-AMP-activated protein kinase catalytic subunit alpha-1",
  "gene_symbol": "PRKAA1",
  "term_id": "GO:1904262",
  "term_label": "negative regulation of TORC1 signaling"
}